type III transforming growth factor beta receptor binding [GO:0034714] (molecular function) Sources: GOC:BHF, GOC:mah Also known as: TGF-beta type III binding, transforming growth factor beta receptor type III binding, type IIII TGF-beta binding, betaglycan binding, transforming growth factor beta ligand binding to type III receptor Definition: Binding to a type III transforming growth factor beta receptor. Relationships: is a type of transforming growth factor beta receptor binding [GO:0005160]